{
  "term_label": "Unknown cellular component",
  "gene_symbol": "LINC02901",
  "term_id": "UNKNOWN:0003",
  "gene": "UniProtKB:Q4VX62",
  "gene_name": "Putative uncharacterized protein LINC02901"
}